phosphatidic acid biosynthetic process [GO:0006654] (biological process) Relationships: is a type of phosphatidic acid metabolic process [GO:0046473]; is a type of glycerophospholipid biosynthetic process [GO:0046474] Also known as: phosphatidic acid anabolism, phosphatidic acid biosynthesis, phosphatidic acid formation, phosphatidic acid synthesis Sources: ISBN:0198506732 Regulation: regulated by regulation of phosphatidic acid biosynthetic process [GO:1905693]; negatively regulated by GO:1905694; positively regulated by positive regulation of phosphatidic acid biosynthetic process [GO:1905695] Definition: The chemical reactions and pathways resulting in the formation of phosphatidic acid, any derivative of glycerol phosphate in which both the remaining hydroxyl groups of the glycerol moiety are esterified with fatty acids.